{
  "term_label": "canonical Wnt signaling pathway",
  "term_id": "GO:0060070",
  "gene_name": "Frizzled-2",
  "gene": "UniProtKB:Q14332",
  "gene_symbol": "FZD2"
}